{
  "gene_symbol": "TOR4A",
  "term_id": "UNKNOWN:0002",
  "gene": "UniProtKB:Q9NXH8",
  "gene_name": "Torsin-4A",
  "term_label": "Unknown biological process"
}